regulation of autophagosome size [GO:0016243] (biological process) Also known as: regulation of autophagic vacuole size Relationships: is a type of GO:0032535; is_a GO:1905037 Definition: Any process that modulates the size of the autophagosome. Subtypes: negative regulation of autophagosome size [GO:0045771], positive regulation of autophagosome size [GO:0045772] Sources: GOC:autophagy, GOC:krc